{
  "gene": "UniProtKB:O14896",
  "term_id": "GO:0000981",
  "gene_name": "Interferon regulatory factor 6",
  "term_label": "DNA-binding transcription factor activity, RNA polymerase II-specific",
  "gene_symbol": "IRF6"
}